amide metabolic process [GO:0043603] (biological process) Relationships: is a type of GO:0008152 Also known as: amide metabolism, cellular amide metabolic process Definition: The chemical reactions and pathways involving an amide, any derivative of an oxoacid in which an acidic hydroxy group has been replaced by an amino or substituted amino group, as carried out by individual cells. Regulation: regulated by regulation of amide metabolic process [GO:0034248]; negatively regulated by negative regulation of amide metabolic process [GO:0034249]; positively regulated by positive regulation of amide metabolic process [GO:0034250] Note: Note that this term is in the subset of terms that should not be used for direct gene product annotation. Instead, select a child term or, if no appropriate child term exists, please request a new term. Direct annotations to this term may be amended during annotation QC. Sources: GOC:curators Subtypes: allantoin metabolic process [GO:0000255], pyoverdine catabolic process [GO:0002050], GO:0006054, GO:0006637, ceramide metabolic process [GO:0006672], sphingomyelin metabolic process [GO:0006684], glutathione metabolic process [GO:0006749], biotin metabolic process [GO:0006768], nicotinamide metabolic process [GO:0006769], GO:0009050, ureide catabolic process [GO:0010136], substance P catabolic process [GO:0010814], bradykinin catabolic process [GO:0010815], calcitonin catabolic process [GO:0010816], coenzyme A metabolic process [GO:0015936], pantothenate metabolic process [GO:0015939], peptide hormone processing [GO:0016486], iprodione metabolic process [GO:0018922], vibriobactin metabolic process [GO:0019536], GO:0019627, GO:0030186, peptide antibiotic catabolic process [GO:0030652], carnosine metabolic process [GO:0035498], chrysobactin catabolic process [GO:0042859], achromobactin catabolic process [GO:0042862], amide biosynthetic process [GO:0043604], amide catabolic process [GO:0043605], bacteriocin metabolic process [GO:0046224], 2-chloro-N-isopropylacetanilide catabolic process [GO:0046302], GO:0046655, phytochelatin metabolic process [GO:0046937], amyloid-beta metabolic process [GO:0050435], GO:0050761, dihydrolipoamide metabolic process [GO:0051068], GO:0062126, N-acylphosphatidylethanolamine metabolic process [GO:0070292], L-asparagine metabolic process [GO:0070982], lactam metabolic process [GO:0072338], tensidol A catabolic process [GO:1900604], tensidol B catabolic process [GO:1900607], GO:1900817, bacitracin A catabolic process [GO:1901123], leukotriene D4 catabolic process [GO:1901749], lincomycin catabolic process [GO:1901773], GO:2001309